chromatin binding [GO:0003682] (molecular function) Subtypes: chromatin DNA binding [GO:0031490], GO:0031491, euchromatin binding [GO:1990188], promoter-specific chromatin binding [GO:1990841] Relationships: is a type of GO:0005488 Regulation: negatively regulated by negative regulation of chromatin binding [GO:0035562]; positively regulated by positive regulation of chromatin binding [GO:0035563] Definition: Binding to chromatin, the network of fibers of DNA, protein, and sometimes RNA, that make up the chromosomes of the eukaryotic nucleus during interphase. Also known as: lamin/chromatin binding, microtubule/chromatin interaction, nuclear membrane vesicle binding to chromatin References: PMID:20404130 Sources: GOC:jl, ISBN:0198506732